{
  "term_label": "Golgi organization",
  "gene_name": "Conserved oligomeric Golgi complex subunit 4",
  "gene_symbol": "COG4",
  "term_id": "GO:0007030",
  "gene": "UniProtKB:Q9H9E3"
}